{
  "gene_symbol": "CCDC144NL",
  "term_id": "UNKNOWN:0002",
  "term_label": "Unknown biological process",
  "gene_name": "Putative coiled-coil domain-containing protein 144 N-terminal-like",
  "gene": "UniProtKB:Q6NUI1"
}